detection of electrical stimulus involved in electroception [GO:0050964] (biological process) Relationships: is_a GO:0050963; BFO_0000050 electroception [GO:0050956] Sources: GOC:ai, GOC:dos Also known as: electroception, detection of electrical stimulus, electroception, sensory detection of electrical stimulus, electroception, sensory transduction, electroception, sensory transduction of electrical stimulus, detection of electrical stimulus during electroreception, sensory detection of electrical stimulus during electroception, sensory transduction of electrical stimulus during electroception Definition: The series of events that contribute to electroception in which an electrical stimulus is received and converted into a molecular signal.